{
  "gene_name": "Cadherin-20",
  "gene": "UniProtKB:Q9HBT6",
  "term_label": "adherens junction organization",
  "gene_symbol": "CDH20",
  "term_id": "GO:0034332"
}